{
  "term_label": "peptidase activity",
  "gene_name": "Leishmanolysin-like peptidase",
  "gene_symbol": "LMLN",
  "gene": "UniProtKB:Q96KR4",
  "term_id": "GO:0008233"
}